{
  "gene": "UniProtKB:O95754",
  "term_id": "GO:0030215",
  "gene_name": "Semaphorin-4F",
  "term_label": "semaphorin receptor binding",
  "gene_symbol": "SEMA4F"
}